{
  "gene": "UniProtKB:Q9H9P8",
  "term_id": "GO:0047545",
  "gene_name": "L-2-hydroxyglutarate dehydrogenase, mitochondrial",
  "gene_symbol": "L2HGDH",
  "term_label": "(S)-2-hydroxyglutarate dehydrogenase activity"
}